{
  "gene_symbol": "ZNF672",
  "gene_name": "Zinc finger protein 672",
  "gene": "UniProtKB:Q499Z4",
  "term_id": "GO:0000981",
  "term_label": "DNA-binding transcription factor activity, RNA polymerase II-specific"
}